{
  "term_id": "GO:0043204",
  "term_label": "perikaryon",
  "gene_symbol": "GIGYF2",
  "gene": "UniProtKB:Q6Y7W6",
  "gene_name": "GRB10-interacting GYF protein 2"
}